myosin phosphatase regulator activity [GO:0017020] (molecular function) References: PMID:10491107 Sources: GOC:ai Definition: Binds to and modulates of the activity of myosin phosphatase. Relationships: is a type of protein phosphatase regulator activity [GO:0019888]; RO_0002211 myosin phosphatase activity [GO:0017018] Also known as: myosin phosphatase, intrinsic regulator activity